{
  "gene": "UniProtKB:Q76B58",
  "gene_name": "BMP_retinoic acid-inducible neural-specific protein 3",
  "term_label": "dendrite",
  "gene_symbol": "BRINP3",
  "term_id": "GO:0030425"
}